{
  "gene": "UniProtKB:Q96KX0",
  "term_id": "GO:0036126",
  "gene_name": "Lysozyme-like protein 4",
  "term_label": "sperm flagellum",
  "gene_symbol": "LYZL4"
}